{
  "gene": "UniProtKB:Q8IZS6",
  "term_id": "GO:0045505",
  "term_label": "dynein intermediate chain binding",
  "gene_symbol": "DYNLT2",
  "gene_name": "Dynein light chain Tctex-type protein 2"
}